{
  "term_label": "DNA-binding transcription factor activity, RNA polymerase II-specific",
  "term_id": "GO:0000981",
  "gene_name": "Zinc finger and SCAN domain-containing protein 10",
  "gene": "UniProtKB:Q96SZ4",
  "gene_symbol": "ZSCAN10"
}